{
  "term_id": "UNKNOWN:0002",
  "gene_symbol": "TMEM132D",
  "gene_name": "Transmembrane protein 132D",
  "term_label": "Unknown biological process",
  "gene": "UniProtKB:Q14C87"
}